histamine-induced gastric acid secretion [GO:0001697] (biological process) Relationships: is a type of gastric acid secretion [GO:0001696] Sources: GOC:hjd Definition: The regulated release of gastric acid induced by the interaction of histamine with H2 type receptor receptors with subsequent activation of adenylate cyclase and elevation of intracellular cyclic AMP.